{
  "gene_symbol": "DIPK1C",
  "term_id": "UNKNOWN:0003",
  "term_label": "Unknown cellular component",
  "gene": "UniProtKB:Q0P6D2",
  "gene_name": "Divergent protein kinase domain 1C"
}